{
  "gene": "UniProtKB:Q0VDF9",
  "term_id": "GO:0005634",
  "gene_symbol": "HSPA14",
  "gene_name": "Heat shock 70 kDa protein 14",
  "term_label": "nucleus"
}